{
  "gene_name": "C-X-C chemokine receptor type 1",
  "gene_symbol": "CXCR1",
  "term_label": "calcium-mediated signaling",
  "gene": "UniProtKB:P25024",
  "term_id": "GO:0019722"
}